{
  "gene_name": "ADP-ribosylation factor-like protein 6-interacting protein 4",
  "gene": "UniProtKB:Q66PJ3",
  "term_label": "Unknown cellular component",
  "term_id": "UNKNOWN:0003",
  "gene_symbol": "ARL6IP4"
}